muscle cell development [GO:0055001] (biological process) Relationships: is a type of GO:0048468; BFO_0000050 muscle cell differentiation [GO:0042692] Sources: CL:0000187, GOC:devbiol Subtypes: striated muscle cell development [GO:0055002], GO:0097084 Also known as: muscle fiber development, muscle fibre development, myofiber development, myofibre development Definition: The process whose specific outcome is the progression of a muscle cell over time, from its formation to the mature structure. Muscle cell development does not include the steps involved in committing an unspecified cell to the muscle cell fate.